clathrin-coated vesicle [GO:0030136] (cellular component) Definition: A vesicle with a coat formed of clathrin connected to the membrane via one of the clathrin adaptor complexes. References: PMID:11252894 Sources: GOC:mah Relationships: is a type of coated vesicle [GO:0030135] Subtypes: trans-Golgi network transport vesicle [GO:0030140], Weibel-Palade body [GO:0033093], clathrin-coated endocytic vesicle [GO:0045334], GO:0060198